{
  "gene_symbol": "SLC11A1",
  "term_label": "manganese ion transport",
  "gene": "UniProtKB:P49279",
  "term_id": "GO:0006828",
  "gene_name": "Natural resistance-associated macrophage protein 1"
}